positive regulation of pyrimidine nucleotide biosynthetic process [GO:1900399] (biological process) Sources: GOC:TermGenie Relationships: is a type of positive regulation of nucleotide biosynthetic process [GO:0030810]; is a type of regulation of pyrimidine nucleotide biosynthetic process [GO:1900397]; positively regulates pyrimidine nucleotide biosynthetic process [GO:0006221] Definition: Any process that activates or increases the frequency, rate or extent of pyrimidine nucleotide biosynthetic process. Also known as: activation of pyrimidine nucleotide anabolism, activation of pyrimidine nucleotide biosynthesis, activation of pyrimidine nucleotide formation, activation of pyrimidine nucleotide synthesis, positive regulation of pyrimidine nucleotide anabolism, positive regulation of pyrimidine nucleotide biosynthesis, positive regulation of pyrimidine nucleotide formation, positive regulation of pyrimidine nucleotide synthesis, up regulation of pyrimidine nucleotide anabolism, up regulation of pyrimidine nucleotide biosynthesis, up regulation of pyrimidine nucleotide biosynthetic process, up regulation of pyrimidine nucleotide formation, up regulation of pyrimidine nucleotide synthesis, up-regulation of pyrimidine nucleotide anabolism, up-regulation of pyrimidine nucleotide biosynthesis, up-regulation of pyrimidine nucleotide biosynthetic process, up-regulation of pyrimidine nucleotide formation, up-regulation of pyrimidine nucleotide synthesis, upregulation of pyrimidine nucleotide anabolism, upregulation of pyrimidine nucleotide biosynthesis, upregulation of pyrimidine nucleotide biosynthetic process, upregulation of pyrimidine nucleotide formation, upregulation of pyrimidine nucleotide synthesis, activation of pyrimidine nucleotide biosynthetic process